{
  "term_id": "GO:0003950",
  "term_label": "NAD+ poly-ADP-ribosyltransferase activity",
  "gene_symbol": "PARP15",
  "gene": "UniProtKB:Q460N3",
  "gene_name": "Protein mono-ADP-ribosyltransferase PARP15"
}